{
  "gene_name": "Uncharacterized protein",
  "gene": "UniProtKB:A0A494C1I1",
  "gene_symbol": "LOC728392",
  "term_id": "UNKNOWN:0001",
  "term_label": "Unknown molecular function"
}